{
  "gene_name": "G antigen 10",
  "gene_symbol": "GAGE10",
  "term_label": "Unknown biological process",
  "gene": "UniProtKB:A6NGK3",
  "term_id": "UNKNOWN:0002"
}